{
  "term_id": "GO:0030971",
  "gene_name": "ALK and LTK ligand 1",
  "gene_symbol": "ALKAL1",
  "term_label": "receptor tyrosine kinase binding",
  "gene": "UniProtKB:Q6UXT8"
}